{
  "gene": "UniProtKB:P29033",
  "gene_name": "Gap junction beta-2 protein",
  "term_id": "GO:0005243",
  "term_label": "gap junction channel activity",
  "gene_symbol": "GJB2"
}